milk ejection reflex [GO:0060156] (biological process) Definition: A reflex that occurs in response to suckling, beginning with a nerve impulse from a receptor in the mammary gland and ending with the ejection of milk from the gland. Signaling never reaches a level of consciousness. Also known as: milk ejection Sources: GOC:cjm, GOC:dph, GOC:mr, GOC:st Relationships: is a type of body fluid secretion [GO:0007589]; is a type of secretion by tissue [GO:0032941]; is_a reflex [GO:0060004]; is part of lactation [GO:0007595]